{
  "term_label": "Unknown cellular component",
  "gene_symbol": "LCE1C",
  "term_id": "UNKNOWN:0003",
  "gene": "UniProtKB:Q5T751",
  "gene_name": "Late cornified envelope protein 1C"
}